phosphatidylserine exposure on osteoblast involved in bone mineralization [GO:0061592] (biological process) Relationships: is a type of plasma membrane phospholipid scrambling [GO:0017121]; is part of GO:0030282 References: PMID:22936354 Sources: GOC:krc Definition: A phospholipid scrambling process that results in the appearance of phosphatidylserine on the surface of osteoblasts, and contributes to bone mineralization.